{
  "gene_name": "VPS10 domain-containing receptor SorCS3",
  "gene_symbol": "SORCS3",
  "gene": "UniProtKB:Q9UPU3",
  "term_label": "transmembrane signaling receptor activity",
  "term_id": "GO:0004888"
}